{
  "term_id": "GO:0004674",
  "term_label": "protein serine/threonine kinase activity",
  "gene": "UniProtKB:O94804",
  "gene_symbol": "STK10",
  "gene_name": "Serine_threonine-protein kinase 10"
}